negative regulation of clathrin-dependent endocytosis [GO:1900186] (biological process) Definition: Any process that stops, prevents or reduces the frequency, rate or extent of clathrin-mediated endocytosis. Sources: GOC:TermGenie Also known as: down regulation of clathrin coated pit-dependent endocytosis, down regulation of clathrin-dependent endocytosis, down regulation of clathrin-mediated endocytosis, down-regulation of clathrin coated pit-dependent endocytosis, down-regulation of clathrin-dependent endocytosis, down-regulation of clathrin-mediated endocytosis, downregulation of clathrin coated pit-dependent endocytosis, downregulation of clathrin-dependent endocytosis, downregulation of clathrin-mediated endocytosis, inhibition of clathrin coated pit-dependent endocytosis, inhibition of clathrin-dependent endocytosis, negative regulation of clathrin coated pit-dependent endocytosis, negative regulation of clathrin-mediated endocytosis, inhibition of clathrin-mediated endocytosis Relationships: is a type of negative regulation of receptor-mediated endocytosis [GO:0048261]; is a type of regulation of clathrin-dependent endocytosis [GO:2000369]; negatively regulates clathrin-dependent endocytosis [GO:0072583]